{
  "gene_name": "Translocation protein SEC62",
  "term_label": "post-translational protein targeting to membrane, translocation",
  "gene": "UniProtKB:Q99442",
  "term_id": "GO:0031204",
  "gene_symbol": "SEC62"
}